DNA repair [GO:0006281] (biological process) Regulation: regulated by regulation of DNA repair [GO:0006282]; RO_0002212 by negative regulation of DNA repair [GO:0045738]; RO_0002213 by positive regulation of DNA repair [GO:0045739] Subtypes: GO:0000012, recombinational repair [GO:0000725], base-excision repair [GO:0006284], nucleotide-excision repair [GO:0006289], pyrimidine dimer repair [GO:0006290], mismatch repair [GO:0006298], GO:0006302, DNA alkylation repair [GO:0006307], non-photoreactive DNA repair [GO:0010213], interstrand cross-link repair [GO:0036297], GO:0043504, GO:0045004, viral DNA repair [GO:0046787], UV-damage excision repair [GO:0070914], GO:0106300, chromosomal 5-methylcytosine DNA demethylation, oxidative deamination pathway [GO:0141168] Definition: The process of restoring DNA after damage. Genomes are subject to damage by chemical and physical agents in the environment (e.g. UV and ionizing radiations, chemical mutagens, fungal and bacterial toxins, etc.) and by free radicals or alkylating agents endogenously generated in metabolism. DNA is also damaged because of errors during its replication. A variety of different DNA repair pathways have been reported that include direct reversal, base excision repair, nucleotide excision repair, photoreactivation, bypass, double-strand break repair pathway, and mismatch repair pathway. Relationships: is_a GO:0006259; is a type of DNA damage response [GO:0006974] References: PMID:11563486